{
  "term_label": "Unknown cellular component",
  "gene_symbol": "FRG2",
  "term_id": "UNKNOWN:0003",
  "gene_name": "Protein FRG2",
  "gene": "UniProtKB:Q64ET8"
}